guard cell differentiation [GO:0010052] (biological process) Definition: The process in which a guard mother cell acquires the specialized features of a guard cell. Sources: GOC:expert_db, GOC:tb Also known as: stomatal cell differentiation Relationships: is a type of plant epidermal cell differentiation [GO:0090627]; is part of GO:0010103